{
  "gene_symbol": "FEZ1",
  "gene": "UniProtKB:Q99689",
  "term_id": "GO:0030424",
  "gene_name": "Fasciculation and elongation protein zeta-1",
  "term_label": "axon"
}